cytokine receptor binding [GO:0005126] (molecular function) Definition: Binding to a cytokine receptor. Sources: GOC:mah, GOC:vw Also known as: hematopoietin/interferon-class (D200-domain) cytokine receptor binding, hematopoietin/interferon-class (D200-domain) cytokine receptor ligand Relationships: is a type of GO:0005102 Subtypes: interleukin-21 receptor binding [GO:0001531], interleukin-33 receptor binding [GO:0002112], ciliary neurotrophic factor receptor binding [GO:0005127], erythropoietin receptor binding [GO:0005128], granulocyte macrophage colony-stimulating factor receptor binding [GO:0005129], granulocyte colony-stimulating factor receptor binding [GO:0005130], growth hormone receptor binding [GO:0005131], type I interferon receptor binding [GO:0005132], type II interferon receptor binding [GO:0005133], interleukin-2 receptor binding [GO:0005134], GO:0005135, GO:0005136, GO:0005137, interleukin-6 receptor binding [GO:0005138], interleukin-7 receptor binding [GO:0005139], interleukin-9 receptor binding [GO:0005140], interleukin-10 receptor binding [GO:0005141], interleukin-11 receptor binding [GO:0005142], GO:0005143, interleukin-13 receptor binding [GO:0005144], GO:0005146, oncostatin-M receptor binding [GO:0005147], prolactin receptor binding [GO:0005148], GO:0005149, interleukin-1 receptor antagonist activity [GO:0005152], macrophage colony-stimulating factor receptor binding [GO:0005157], transforming growth factor beta receptor binding [GO:0005160], neurotrophin receptor binding [GO:0005165], vascular endothelial growth factor receptor binding [GO:0005172], stem cell factor receptor binding [GO:0005173], interleukin-15 receptor binding [GO:0016170], interleukin-17 receptor binding [GO:0030367], GO:0030380, interleukin-28 receptor binding [GO:0032003], tumor necrosis factor receptor superfamily binding [GO:0032813], chemokine receptor binding [GO:0042379], interleukin-16 receptor binding [GO:0045514], GO:0045515, interleukin-19 receptor binding [GO:0045516], interleukin-20 receptor binding [GO:0045517], interleukin-22 receptor binding [GO:0045518], GO:0045519, interleukin-24 receptor binding [GO:0045520], interleukin-25 receptor binding [GO:0045521], GO:0045522, interleukin-27 receptor binding [GO:0045523], GO:0070748